{
  "gene_symbol": "MMP15",
  "gene": "UniProtKB:P51511",
  "gene_name": "Matrix metalloproteinase-15",
  "term_label": "metalloendopeptidase activity",
  "term_id": "GO:0004222"
}